metanephric collecting duct development [GO:0072205] (biological process) Relationships: is a type of collecting duct development [GO:0072044]; is part of metanephros development [GO:0001656] Sources: GOC:mtg_kidney_jan10 Definition: The process whose specific outcome is the progression of a collecting duct in the metanephros over time, from its formation to the mature structure. The collecting duct responds to vasopressin and aldosterone to regulate water, electrolyte and acid-base balance. The collecting duct is the final common path through which urine flows before entering the ureter and then emptying into the bladder.